intracellular sterol transport [GO:0032366] (biological process) Sources: GOC:mah Relationships: is a type of sterol transport [GO:0015918]; is_a intracellular lipid transport [GO:0032365] Regulation: regulated by regulation of intracellular sterol transport [GO:0032380]; negatively regulated by GO:0032381; positively regulated by GO:0032382 Definition: The directed movement of sterols within cells. Subtypes: intracellular cholesterol transport [GO:0032367]